{
  "term_id": "GO:0005737",
  "gene_symbol": "JMJD4",
  "gene": "UniProtKB:Q9H9V9",
  "gene_name": "2-oxoglutarate and iron-dependent oxygenase JMJD4",
  "term_label": "cytoplasm"
}